{
  "gene_name": "Solute carrier organic anion transporter family member 1B1",
  "term_id": "GO:0015125",
  "gene": "UniProtKB:Q9Y6L6",
  "term_label": "bile acid transmembrane transporter activity",
  "gene_symbol": "SLCO1B1"
}